pollen development [GO:0009555] (biological process) Sources: GOC:mtg_plant, GOC:mtg_sensu, GOC:tb Also known as: formation of generative and vegetative cells, male gametophyte development, male gametophyte formation, microgametophyte development, pollen grain formation Relationships: is a type of gametophyte development [GO:0048229]; has part microsporogenesis [GO:0009556] Definition: The process whose specific outcome is the progression of the pollen grain over time, from its formation to the mature structure. The process begins with the meiosis of the microsporocyte to form four haploid microspores. The nucleus of each microspore then divides by mitosis to form a two-celled organism, the pollen grain, that contains a tube cell as well as a smaller generative cell. The pollen grain is surrounded by an elaborate cell wall. In some species, the generative cell immediately divides again to give a pair of sperm cells. In most flowering plants, however this division takes place later, in the tube that develops when a pollen grain germinates.